{
  "gene_name": "Golgi to ER traffic protein 4 homolog",
  "term_label": "BAT3 complex",
  "gene": "UniProtKB:Q7L5D6",
  "gene_symbol": "GET4",
  "term_id": "GO:0071818"
}